{
  "gene_name": "Myelodysplastic syndrome 2 translocation-associated protein",
  "term_id": "UNKNOWN:0001",
  "term_label": "Unknown molecular function",
  "gene_symbol": "MDS2",
  "gene": "UniProtKB:Q8NDY4"
}